{
  "gene": "UniProtKB:P30304",
  "gene_name": "M-phase inducer phosphatase 1",
  "term_id": "GO:0110032",
  "gene_symbol": "CDC25A",
  "term_label": "positive regulation of G2/MI transition of meiotic cell cycle"
}